{
  "term_label": "Unknown biological process",
  "term_id": "UNKNOWN:0002",
  "gene_name": "Acid ceramidase",
  "gene": "UniProtKB:Q13510",
  "gene_symbol": "ASAH1"
}